{
  "term_id": "UNKNOWN:0003",
  "term_label": "Unknown cellular component",
  "gene": "UniProtKB:Q8TF61",
  "gene_symbol": "FBXO41",
  "gene_name": "F-box only protein 41"
}